{
  "gene": "UniProtKB:Q15256",
  "gene_name": "Receptor-type tyrosine-protein phosphatase R",
  "gene_symbol": "PTPRR",
  "term_label": "protein kinase binding",
  "term_id": "GO:0019901"
}